{
  "term_id": "GO:0005886",
  "gene_symbol": "CPN2",
  "gene_name": "Carboxypeptidase N subunit 2",
  "gene": "UniProtKB:P22792",
  "term_label": "plasma membrane"
}